tRNA methyltransferase activity [GO:0008175] (molecular function) Sources: GOC:mah Definition: Catalysis of the transfer of a methyl group from a donor to a nucleoside residue in a tRNA molecule. Subtypes: GO:0016300, tRNA (guanine) methyltransferase activity [GO:0016423], GO:0016426, tRNA (cytidine) methyltransferase activity [GO:0016427], GO:0106050 Relationships: is a type of GO:0008173; is_a catalytic activity, acting on a tRNA [GO:0140101]